SMAD binding [GO:0046332] (molecular function) Subtypes: co-SMAD binding [GO:0070410], I-SMAD binding [GO:0070411], R-SMAD binding [GO:0070412] Relationships: is a type of protein binding [GO:0005515] Sources: GOC:ai Definition: Binding to a SMAD signaling protein.